{
  "gene": "UniProtKB:Q86UE3",
  "gene_symbol": "ZNF546",
  "term_id": "GO:0005634",
  "gene_name": "Zinc finger protein 546",
  "term_label": "nucleus"
}